{
  "gene_symbol": "LIMD2",
  "term_label": "actin filament bundle assembly",
  "gene": "UniProtKB:Q9BT23",
  "gene_name": "LIM domain-containing protein 2",
  "term_id": "GO:0051017"
}